regulation of encysted zoospore germination [GO:0075227] (biological process) Sources: GOC:pamgo_curators Definition: Any process that modulates the frequency, rate or extent of an encysted zoospore germination. Relationships: is a type of regulation of spore germination [GO:1904359]; regulates encysted zoospore germination [GO:0075226] Subtypes: positive regulation of encysted zoospore germination [GO:0075228], negative regulation of encysted zoospore germination [GO:0075229] Also known as: modulation of encysted zoospore germination on or near host, regulation of encysted zoospore germination on or near host